{
  "gene_name": "Tumor protein p73",
  "term_label": "nucleus",
  "gene": "UniProtKB:O15350",
  "term_id": "GO:0005634",
  "gene_symbol": "TP73"
}